{
  "term_id": "GO:0005549",
  "gene": "UniProtKB:Q8NHC6",
  "term_label": "odorant binding",
  "gene_symbol": "OR14L1",
  "gene_name": "Olfactory receptor 14L1"
}